{
  "gene_symbol": "BTG2",
  "gene_name": "Protein BTG2",
  "term_label": "nucleus",
  "term_id": "GO:0005634",
  "gene": "UniProtKB:P78543"
}